{
  "gene": "UniProtKB:P30049",
  "term_id": "GO:0046933",
  "term_label": "proton-transporting ATP synthase activity, rotational mechanism",
  "gene_symbol": "ATP5F1D",
  "gene_name": "ATP synthase subunit delta, mitochondrial"
}